{
  "gene": "UniProtKB:Q7Z7G2",
  "gene_name": "Complexin-4",
  "term_id": "GO:0043195",
  "term_label": "terminal bouton",
  "gene_symbol": "CPLX4"
}